{
  "gene": "UniProtKB:Q93008",
  "term_id": "GO:0004843",
  "gene_symbol": "USP9X",
  "gene_name": "Probable ubiquitin carboxyl-terminal hydrolase FAF-X",
  "term_label": "cysteine-type deubiquitinase activity"
}